positive regulation of cholesterol biosynthetic process [GO:0045542] (biological process) Relationships: is_a regulation of cholesterol biosynthetic process [GO:0045540]; is a type of GO:0090205; is a type of GO:0106120; is a type of positive regulation of alcohol biosynthetic process [GO:1902932]; positively regulates cholesterol biosynthetic process [GO:0006695] Sources: GOC:go_curators Definition: Any process that activates or increases the frequency, rate or extent of the chemical reactions and pathways resulting in the formation of cholesterol. Also known as: positive regulation of cholesterol anabolism, positive regulation of cholesterol biosynthesis, positive regulation of cholesterol formation, positive regulation of cholesterol synthesis, up regulation of cholesterol biosynthetic process, up-regulation of cholesterol biosynthetic process, upregulation of cholesterol biosynthetic process, activation of cholesterol biosynthetic process, stimulation of cholesterol biosynthetic process